{
  "term_id": "GO:0005132",
  "gene": "UniProtKB:P01562",
  "gene_symbol": "IFNA1",
  "gene_name": "Interferon alpha-1_13",
  "term_label": "type I interferon receptor binding"
}